{
  "gene_symbol": "GRN",
  "gene": "UniProtKB:P28799",
  "term_label": "regulation of inflammatory response",
  "term_id": "GO:0050727",
  "gene_name": "Progranulin"
}